developmental growth [GO:0048589] (BP) Definition: The increase in size or mass of an entire organism, a part of an organism or a cell, where the increase in size or mass has the specific outcome of the progression of the organism over time from one condition to another. Subtypes: primary ovarian follicle growth [GO:0001545], preantral ovarian follicle growth [GO:0001546], antral ovarian follicle growth [GO:0001547], ovarian cumulus expansion [GO:0001550], blastocyst growth [GO:0001832], heart capillary growth [GO:0003248], growth of a germarium-derived egg chamber [GO:0007295], imaginal disc growth [GO:0007446], multicellular organism growth [GO:0035264], organ growth [GO:0035265], meristem growth [GO:0035266], tissue regeneration [GO:0042246], uterine wall growth [GO:0042702], developmental cell growth [GO:0048588], skeletal muscle tissue growth [GO:0048630], synaptic assembly at neuromuscular junction [GO:0051124], cardiac muscle tissue growth [GO:0055017], developmental growth involved in morphogenesis [GO:0060560], seed growth [GO:0080112], developmental vegetative growth [GO:0080186], GO:0090214 Sources: GOC:go_curators Regulation: regulated by regulation of developmental growth [GO:0048638]; positively regulated by positive regulation of developmental growth [GO:0048639]; negatively regulated by GO:0048640 Relationships: is a type of growth [GO:0040007]; is part of developmental process [GO:0032502]